troponin T binding [GO:0031014] (molecular function) Definition: Binding to troponin T, the tropomyosin-binding subunit of the troponin complex. Sources: GOC:mah, ISBN:0815316194 Relationships: is_a cytoskeletal protein binding [GO:0008092]